{
  "gene_symbol": "CNGA1",
  "gene_name": "cGMP-gated cation channel alpha-1",
  "term_label": "intracellular cyclic nucleotide activated cation channel complex",
  "gene": "UniProtKB:P29973",
  "term_id": "GO:0017071"
}